{
  "gene_name": "Proprotein convertase subtilisin_kexin type 4",
  "term_label": "trans-Golgi network",
  "term_id": "GO:0005802",
  "gene": "UniProtKB:Q6UW60",
  "gene_symbol": "PCSK4"
}